peptide noradrenalinyltransferase activity [GO:0120298] (molecular function) Definition: Catalysis of the reaction: (R)-noradrenaline + L-glutaminyl-[protein] = 5-(R)-noradrenalinyl-L-glutamyl-[protein] + NH4(+). References: PMID:22858378 Sources: GOC:sp Relationships: is a type of N-acyltransferase activity [GO:0016410]